potassium:sodium symporter activity [GO:0009674] (molecular function) Subtypes: GO:0008511 Definition: Enables the transfer of a solute or solutes from one side of a membrane to the other according to the reaction: K+(out) + Na+(out) = K+(in) + Na+(in). Also known as: high affinity potassium transporter Relationships: is a type of GO:0015079; is a type of solute:sodium symporter activity [GO:0015370] Sources: TC:2.A.38.3.1